{
  "gene": "UniProtKB:Q8NBW4",
  "term_id": "GO:0005765",
  "term_label": "lysosomal membrane",
  "gene_name": "Neutral amino acid transporter 9",
  "gene_symbol": "SLC38A9"
}